{
  "term_label": "nucleolus",
  "gene_symbol": "RRP36",
  "gene_name": "Ribosomal RNA processing protein 36 homolog",
  "gene": "UniProtKB:Q96EU6",
  "term_id": "GO:0005730"
}